{
  "term_id": "GO:0005615",
  "gene": "UniProtKB:O43300",
  "gene_symbol": "LRRTM2",
  "term_label": "extracellular space",
  "gene_name": "Leucine-rich repeat transmembrane neuronal protein 2"
}